{
  "gene_symbol": "AMOTL2",
  "gene_name": "Angiomotin-like protein 2",
  "gene": "UniProtKB:Q9Y2J4",
  "term_id": "GO:0005923",
  "term_label": "bicellular tight junction"
}